{
  "gene_name": "Anaphase-promoting complex subunit 5",
  "gene_symbol": "ANAPC5",
  "gene": "UniProtKB:Q9UJX4",
  "term_id": "GO:0045842",
  "term_label": "positive regulation of mitotic metaphase/anaphase transition"
}